{
  "gene_symbol": "FOXC2",
  "term_id": "GO:0000981",
  "gene_name": "Forkhead box protein C2",
  "term_label": "DNA-binding transcription factor activity, RNA polymerase II-specific",
  "gene": "UniProtKB:Q99958"
}